{
  "gene": "UniProtKB:P08567",
  "gene_symbol": "PLEK",
  "term_id": "GO:0030036",
  "term_label": "actin cytoskeleton organization",
  "gene_name": "Pleckstrin"
}